aspartate metabolic process [GO:0006531] (biological process) Sources: GOC:go_curators, ISBN:0198506732 Subtypes: aspartate biosynthetic process [GO:0006532], L-aspartate catabolic process [GO:0006533], GO:0019550, 'de novo' NAD+ biosynthetic process from L-aspartate [GO:0034628] Also known as: aspartate metabolism Definition: The chemical reactions and pathways involving aspartate, the anion derived from aspartic acid, 2-aminobutanedioic acid. Relationships: is a type of dicarboxylic acid metabolic process [GO:0043648]; is a type of GO:1901605